{
  "gene": "UniProtKB:P28223",
  "gene_name": "5-hydroxytryptamine receptor 2A",
  "gene_symbol": "HTR2A",
  "term_label": "chemical synaptic transmission",
  "term_id": "GO:0007268"
}